steryl-beta-glucosidase activity [GO:0050295] (molecular function) Also known as: steryl-b-glucosidase activity, cholesteryl-beta-D-glucoside glucohydrolase activity Definition: Catalysis of the reaction: cholesteryl-beta-D-glucoside + H2O = D-glucose + cholesterol. Sources: EC:3.2.1.104, RHEA:11956 Relationships: is a type of GO:0008422